{
  "term_label": "negative regulation of transcription by RNA polymerase II",
  "gene_symbol": "SOX14",
  "gene": "UniProtKB:O95416",
  "term_id": "GO:0000122",
  "gene_name": "Transcription factor SOX-14"
}